positive regulation of high-density lipoprotein particle clearance [GO:0010983] (biological process) Definition: Any process that increases the rate, frequency or extent of high-density lipoprotein particle clearance. High-density lipoprotein particle clearance is the process in which a high-density lipoprotein particle is removed from the blood via receptor-mediated endocytosis and its constituent parts degraded. Sources: GOC:BHF, GOC:dph, GOC:tb Relationships: is a type of regulation of high-density lipoprotein particle clearance [GO:0010982]; is a type of positive regulation of lipoprotein particle clearance [GO:0010986]; positively regulates GO:0034384